positive regulation of androstenedione secretion [GO:2000839] (biological process) Also known as: positive regulation of androst-4-ene-3,17-dione secretion Relationships: is_a positive regulation of lipid transport [GO:0032370]; is a type of positive regulation of hormone secretion [GO:0046887]; is a type of regulation of androstenedione secretion [GO:2000837]; positively regulates GO:0035941 Sources: GOC:sl Definition: Any process that activates or increases the frequency, rate or extent of androstenedione secretion.